mating-type P-factor pheromone receptor activity [GO:0036320] (molecular function) Definition: Combining with the mating-type peptide pheromone P-factor and transmitting the signal across the membrane to initiate a change in cell activity. P-factor is a polypeptide of 23 residues, with the sequence Thr-Tyr-Ala-Asp-Phe-Leu-Arg-Ala-Tyr-Gln-Ser-Trp-Asn-Thr-Phe-Val-Asn-Pro-Asp-Arg-Pro-Asn-Leu, and is a peptide pheromone released by Schizosaccharomyces pombe cells of the cellular mating type Plus. Relationships: is a type of mating-type factor pheromone receptor activity [GO:0004932]; is a type of peptide pheromone receptor activity [GO:0036318] Also known as: P-factor mating pheromone receptor activity, P-factor receptor activity References: PMID:8314086 Sources: GOC:al